{
  "term_label": "RNA polymerase II transcription regulatory region sequence-specific DNA binding",
  "gene": "UniProtKB:Q68DE3",
  "gene_name": "Basic helix-loop-helix domain-containing protein USF3",
  "term_id": "GO:0000977",
  "gene_symbol": "USF3"
}